neurotrophin p75 receptor binding [GO:0005166] (molecular function) Definition: Binding to a neurotrophin p75 receptor. Sources: GOC:ai Relationships: is a type of neurotrophin receptor binding [GO:0005165] Also known as: neurotrophin p75 receptor ligand